{
  "term_label": "nucleus",
  "gene": "UniProtKB:Q96MF7",
  "term_id": "GO:0005634",
  "gene_name": "E3 SUMO-protein ligase NSE2",
  "gene_symbol": "NSMCE2"
}